{
  "term_label": "plasma membrane",
  "gene_symbol": "ARF4",
  "gene_name": "ADP-ribosylation factor 4",
  "term_id": "GO:0005886",
  "gene": "UniProtKB:P18085"
}